{
  "gene_name": "Cysteine-rich protein 1",
  "term_label": "Unknown cellular component",
  "gene_symbol": "CRIP1",
  "gene": "UniProtKB:P50238",
  "term_id": "UNKNOWN:0003"
}